{
  "gene_name": "Arylsulfatase B",
  "gene_symbol": "ARSB",
  "term_id": "GO:0008484",
  "term_label": "sulfuric ester hydrolase activity",
  "gene": "UniProtKB:P15848"
}